NAD-dependent protein lipoamidase activity [GO:0106419] (molecular function) References: PMID:25525879 Sources: RHEA:63640 Relationships: is a type of GO:0016747 Definition: Catalysis of the reaction: (R)-N6-lipoyl-L-lysyl-[protein] + H2O + NAD+ = 2''-O-lipoyl-ADP-D-ribose + L-lysyl-[protein] + nicotinamide.